{
  "term_id": "GO:0005886",
  "term_label": "plasma membrane",
  "gene_name": "Carcinoembryonic antigen-related cell adhesion molecule 18",
  "gene_symbol": "CEACAM18",
  "gene": "UniProtKB:A8MTB9"
}